cytosolic large ribosomal subunit [GO:0022625] (cellular component) Also known as: 50S ribosomal subunit, 60S ribosomal subunit, eukaryotic ribosomal LSU, prokaryotic large ribosomal subunit Sources: GOC:mtg_sensu Definition: The large subunit of a ribosome located in the cytosol. Relationships: is a type of large ribosomal subunit [GO:0015934]; is part of cytosolic ribosome [GO:0022626]